{
  "gene_symbol": "B2M",
  "term_label": "positive regulation of T cell activation",
  "gene_name": "Beta-2-microglobulin",
  "term_id": "GO:0050870",
  "gene": "UniProtKB:P61769"
}